high-affinity potassium ion transmembrane transporter activity [GO:0140107] (molecular function) References: PMID:10629185 Relationships: is a type of potassium ion transmembrane transporter activity [GO:0015079] Definition: Enables the transfer of potassium ions from one side of a membrane to the other. In high-affinity transport the transporter is able to bind the solute even if it is only present at very low concentrations.